specification of mesonephric tubule identity [GO:0072167] (biological process) Definition: The process in which the tubules of the mesonephros acquire their identity. Sources: GOC:mtg_kidney_jan10 Relationships: is a type of pattern specification involved in mesonephros development [GO:0061227]; is a type of specification of nephron tubule identity [GO:0072081]; is part of mesonephric tubule formation [GO:0072172] Subtypes: specification of anterior mesonephric tubule identity [GO:0072168], specification of posterior mesonephric tubule identity [GO:0072169]